{
  "gene": "UniProtKB:Q4ADV7",
  "term_label": "Ric1-Rgp1 guanyl-nucleotide exchange factor complex",
  "gene_symbol": "RIC1",
  "term_id": "GO:0034066",
  "gene_name": "Guanine nucleotide exchange factor subunit RIC1"
}